siRNA-mediated silent mating type cassette region heterochromatin formation [GO:0140185] (biological process) Definition: The formation of heterochromatin into a heterochromatin domain by a process mediated by a small interfering siRNA at the silent mating-type loci. Also known as: siRNA mediated silent mating type cassette region heterochromatin formation, siRNA-mediated silent-mating type cassette region heterochromatin formation References: PMID:39747188 Relationships: is a type of silent mating-type cassette heterochromatin formation [GO:0030466]; is a type of siRNA-mediated heterochromatin formation [GO:0141194]